negative regulation of interleukin-16 production [GO:0032699] (biological process) Sources: GOC:mah Definition: Any process that stops, prevents, or reduces the frequency, rate, or extent of interleukin-16 production. Also known as: down regulation of interleukin-16 production, down-regulation of interleukin-16 production, downregulation of interleukin-16 production, negative regulation of IL-16 production, inhibition of interleukin-16 production, negative regulation of interleukin-16 biosynthetic process Relationships: is_a negative regulation of cytokine production [GO:0001818]; is a type of GO:0032659; negatively regulates interleukin-16 production [GO:0032619]